{
  "gene_symbol": "SLC25A10",
  "term_label": "sulfate transmembrane transport",
  "gene_name": "Mitochondrial dicarboxylate carrier",
  "gene": "UniProtKB:Q9UBX3",
  "term_id": "GO:1902358"
}